{
  "gene_symbol": "CLDN20",
  "term_label": "bicellular tight junction",
  "gene_name": "Claudin-20",
  "gene": "UniProtKB:P56880",
  "term_id": "GO:0005923"
}